{
  "gene": "UniProtKB:Q5VZ52",
  "term_label": "Unknown molecular function",
  "gene_name": "MORN repeat-containing protein 5",
  "gene_symbol": "MORN5",
  "term_id": "UNKNOWN:0001"
}